{
  "gene_name": "AP2-associated protein kinase 1",
  "term_id": "GO:0004674",
  "gene": "UniProtKB:Q2M2I8",
  "term_label": "protein serine/threonine kinase activity",
  "gene_symbol": "AAK1"
}